{
  "term_label": "Unknown cellular component",
  "gene_symbol": "CCDC182",
  "term_id": "UNKNOWN:0003",
  "gene_name": "Coiled-coil domain-containing protein 182",
  "gene": "UniProtKB:A6NF36"
}